{
  "gene_name": "NADH dehydrogenase [ubiquinone] 1 alpha subcomplex assembly factor 2",
  "term_id": "GO:0032981",
  "gene_symbol": "NDUFAF2",
  "gene": "UniProtKB:Q8N183",
  "term_label": "mitochondrial respiratory chain complex I assembly"
}